{
  "term_label": "protein quality control for misfolded or incompletely synthesized proteins",
  "gene_name": "ATP-dependent zinc metalloprotease YME1L1",
  "gene_symbol": "YME1L1",
  "term_id": "GO:0006515",
  "gene": "UniProtKB:Q96TA2"
}